{
  "gene": "UniProtKB:Q96DX7",
  "gene_symbol": "TRIM44",
  "gene_name": "Tripartite motif-containing protein 44",
  "term_label": "regulation of gene expression",
  "term_id": "GO:0010468"
}